negative regulation of heat dissipation [GO:0031655] (biological process) Sources: GOC:dph, GOC:mah, GOC:tb Also known as: down regulation of heat dissipation, down-regulation of heat dissipation, downregulation of heat dissipation, inhibition of heat dissipation Definition: Any process that stops, prevents, or reduces the rate or extent of heat dissipation. Relationships: is a type of regulation of heat dissipation [GO:0031654]; is_a negative regulation of multicellular organismal process [GO:0051241]; RO_0002212 GO:0031653